{
  "gene": "UniProtKB:A8MV23",
  "gene_name": "Serpin E3",
  "term_id": "UNKNOWN:0002",
  "term_label": "Unknown biological process",
  "gene_symbol": "SERPINE3"
}